{
  "term_label": "bile acid:sodium symporter activity",
  "gene": "UniProtKB:Q12908",
  "gene_name": "Ileal sodium_bile acid cotransporter",
  "term_id": "GO:0008508",
  "gene_symbol": "SLC10A2"
}